{
  "gene_name": "Forkhead box protein R1",
  "gene_symbol": "FOXR1",
  "gene": "UniProtKB:Q6PIV2",
  "term_id": "GO:0005634",
  "term_label": "nucleus"
}